{
  "gene_symbol": "LSM4",
  "term_id": "GO:0017070",
  "gene": "UniProtKB:Q9Y4Z0",
  "gene_name": "U6 snRNA-associated Sm-like protein LSm4",
  "term_label": "U6 snRNA binding"
}